{
  "gene": "UniProtKB:Q86WS4",
  "term_label": "Unknown cellular component",
  "gene_symbol": "C12orf40",
  "gene_name": "Uncharacterized protein C12orf40",
  "term_id": "UNKNOWN:0003"
}